endocardial cushion cell fate specification [GO:0061447] (biological process) Definition: The process involved in the specification of endocardial cushion cell identity. Once specification has taken place, a cell will be committed to differentiate down a specific pathway if left in its normal environment. Relationships: is a type of cardiac cell fate specification [GO:0060912]; is part of endocardial cushion cell fate commitment [GO:0061445] Sources: GOC:BHF, GOC:dph